MutLalpha complex binding [GO:0032405] (molecular function) Relationships: is a type of GO:0032404 Sources: GOC:vk Definition: Binding to a MutLalpha mismatch repair complex.